{
  "gene_symbol": "SMG8",
  "term_label": "Unknown molecular function",
  "gene_name": "Nonsense-mediated mRNA decay factor SMG8",
  "term_id": "UNKNOWN:0001",
  "gene": "UniProtKB:Q8ND04"
}